positive regulation of maltotriulose transport [GO:1900326] (biological process) Sources: GOC:TermGenie, GOC:mengo_curators Relationships: is a type of positive regulation of transport [GO:0051050]; is a type of regulation of maltotriulose transport [GO:1900324]; positively regulates maltotriulose transport [GO:2001090] Also known as: up regulation of maltotriulose transport, up-regulation of maltotriulose transport, upregulation of maltotriulose transport, activation of maltotriulose transport Definition: Any process that activates or increases the frequency, rate or extent of maltotriulose transport.